{
  "term_label": "protein targeting to ER",
  "term_id": "GO:0045047",
  "gene_name": "Signal peptidase complex subunit 1",
  "gene": "UniProtKB:Q9Y6A9",
  "gene_symbol": "SPCS1"
}